{
  "term_label": "Unknown molecular function",
  "gene_symbol": "UBTD2",
  "gene": "UniProtKB:Q8WUN7",
  "gene_name": "Ubiquitin domain-containing protein 2",
  "term_id": "UNKNOWN:0001"
}